{
  "gene_name": "Putative serine protease 42",
  "term_label": "serine-type endopeptidase activity",
  "gene": "UniProtKB:Q7Z5A4",
  "gene_symbol": "PRSS42P",
  "term_id": "GO:0004252"
}